{
  "term_label": "cytosol",
  "gene_symbol": "PMM1",
  "term_id": "GO:0005829",
  "gene_name": "Phosphomannomutase 1",
  "gene": "UniProtKB:Q92871"
}